cerebral cortex cell migration [GO:0021795] (biological process) Definition: The orderly movement of cells from one site to another in the cerebral cortex. Subtypes: cerebral cortex radially oriented cell migration [GO:0021799], cerebral cortex tangential migration [GO:0021800] Relationships: is a type of telencephalon cell migration [GO:0022029]; is part of cerebral cortex development [GO:0021987] Sources: GOC:cls, GOC:dgh, GOC:dph, GOC:jid, GO_REF:0000021